red, far-red light phototransduction [GO:0009585] (biological process) Also known as: phytochrome signaling pathway, red-sensitive opsin Relationships: is a type of phototransduction [GO:0007602]; is part of red or far-red light signaling pathway [GO:0010017] Definition: The sequence of reactions within a cell required to convert absorbed photons from red or far-red light into a molecular signal; the red, far-red light range is defined as having a wavelength within the range 660-730 nm. Sources: GOC:mah